{
  "term_id": "GO:0098839",
  "gene_name": "Metabotropic glutamate receptor 5",
  "term_label": "postsynaptic density membrane",
  "gene": "UniProtKB:P41594",
  "gene_symbol": "GRM5"
}